{
  "term_id": "GO:0090263",
  "gene": "UniProtKB:Q9UGI0",
  "gene_symbol": "ZRANB1",
  "gene_name": "Ubiquitin thioesterase ZRANB1",
  "term_label": "positive regulation of canonical Wnt signaling pathway"
}